{
  "gene": "UniProtKB:Q70EK9",
  "gene_name": "Ubiquitin carboxyl-terminal hydrolase 51",
  "gene_symbol": "USP51",
  "term_label": "Unknown biological process",
  "term_id": "UNKNOWN:0002"
}